negative regulation of triglyceride biosynthetic process [GO:0010868] (biological process) Definition: Any process that decreases the rate, frequency, or extent of triglyceride biosynthesis. Triglyceride biosynthesis is the collection of chemical reactions and pathways resulting in the formation of triglyceride, any triester of glycerol. Relationships: is a type of GO:0010866; is a type of GO:0051055; is a type of negative regulation of triglyceride metabolic process [GO:0090209]; negatively regulates GO:0019432 Also known as: negative regulation of triacylglycerol biosynthetic process Sources: GOC:BHF, GOC:tb